{
  "gene": "UniProtKB:O94850",
  "term_id": "UNKNOWN:0001",
  "term_label": "Unknown molecular function",
  "gene_symbol": "DDN",
  "gene_name": "Dendrin"
}